{
  "gene_symbol": "MAP1LC3C",
  "term_label": "autophagosome membrane",
  "gene": "UniProtKB:Q9BXW4",
  "gene_name": "Microtubule-associated proteins 1A_1B light chain 3C",
  "term_id": "GO:0000421"
}